{
  "gene": "UniProtKB:Q13470",
  "term_id": "GO:0005886",
  "gene_symbol": "TNK1",
  "term_label": "plasma membrane",
  "gene_name": "Non-receptor tyrosine-protein kinase TNK1"
}